aldosterone metabolic process [GO:0032341] (BP) Subtypes: GO:0032342, aldosterone catabolic process [GO:0032343] Regulation: RO_0002211 by regulation of aldosterone metabolic process [GO:0032344] References: PMID:16527843 Also known as: aldosterone metabolism Definition: The chemical reactions and pathways involving aldosterone, a corticosteroid hormone that is produced by the zona glomerulosa of the adrenal cortex and regulates salt (sodium and potassium) and water balance. Relationships: is a type of aldehyde metabolic process [GO:0006081]; is a type of C21-steroid hormone metabolic process [GO:0008207]; is a type of mineralocorticoid metabolic process [GO:0008212]; is a type of primary alcohol metabolic process [GO:0034308]; is a type of ketone metabolic process [GO:0042180]; is a type of olefinic compound metabolic process [GO:0120254]